eukaryotic translation initiation factor 4F complex [GO:0016281] (cellular component) Relationships: is a type of RNA cap binding complex [GO:0034518]; is part of GO:0005737 References: PMID:32883864, PMID:8449919 Sources: GOC:hb Also known as: eukaryotic translation initiation factor 4 complex, cytoplasmic cap-binding complex, eIF-4F Definition: The eukaryotic translation initiation factor 4F complex is composed of eIF4E, eIF4A and eIF4G; it is involved in the recognition of the mRNA cap, ATP-dependent unwinding of the 5'-terminal secondary structure and recruitment of the mRNA to the ribosome.